{
  "term_id": "GO:0002430",
  "gene": "UniProtKB:P21462",
  "gene_symbol": "FPR1",
  "term_label": "complement receptor mediated signaling pathway",
  "gene_name": "fMet-Leu-Phe receptor"
}